{
  "term_id": "GO:0004745",
  "term_label": "all-trans-retinol dehydrogenase (NAD+) activity",
  "gene_name": "All-trans-retinol dehydrogenase [NAD(+)] ADH1B",
  "gene": "UniProtKB:P00325",
  "gene_symbol": "ADH1B"
}